{
  "term_id": "GO:0072344",
  "gene_symbol": "RACK1",
  "term_label": "rescue of stalled ribosome",
  "gene": "UniProtKB:P63244",
  "gene_name": "Small ribosomal subunit protein RACK1"
}